{
  "gene_name": "Neuroblastoma breakpoint family member 1",
  "gene": "UniProtKB:Q3BBV0",
  "term_label": "Unknown cellular component",
  "gene_symbol": "NBPF1",
  "term_id": "UNKNOWN:0003"
}